{
  "gene_symbol": "KRTAP11-1",
  "term_label": "Unknown cellular component",
  "gene_name": "Keratin-associated protein 11-1",
  "gene": "UniProtKB:Q8IUC1",
  "term_id": "UNKNOWN:0003"
}